{
  "term_id": "GO:0005634",
  "term_label": "nucleus",
  "gene_symbol": "GTF2IRD1",
  "gene_name": "General transcription factor II-I repeat domain-containing protein 1",
  "gene": "UniProtKB:Q9UHL9"
}